{
  "gene_name": "Protein argonaute-3",
  "term_label": "single-stranded RNA binding",
  "gene_symbol": "AGO3",
  "term_id": "GO:0003727",
  "gene": "UniProtKB:Q9H9G7"
}